{
  "term_label": "calcium-dependent protein serine/threonine phosphatase regulator activity",
  "term_id": "GO:0008597",
  "gene": "UniProtKB:Q96LZ3",
  "gene_symbol": "PPP3R2",
  "gene_name": "Calcineurin subunit B type 2"
}